contact inhibition [GO:0060242] (biological process) References: PMID:17376520 Sources: GOC:dph Relationships: is_a detection of cell density [GO:0060245] Definition: The series of events in which information about the density of cells in a population is received by direct cell-cell contact and is converted into a molecular signal, resulting in the cessation of cell growth or proliferation. Also known as: detection of cell density by contact stimulus, detection of cell density by contact stimulus involved in contact inhibition